{
  "gene_symbol": "FTMT",
  "term_id": "GO:0008199",
  "gene_name": "Ferritin, mitochondrial",
  "term_label": "ferric iron binding",
  "gene": "UniProtKB:Q8N4E7"
}